positive regulation of intracellular protein transport [GO:0090316] (biological process) Subtypes: GO:0042307, positive regulation of protein export from nucleus [GO:0046827], GO:0070863, positive regulation of protein targeting to vacuolar membrane [GO:1900485], GO:1904053, positive regulation of axo-dendritic protein transport [GO:1905128], positive regulation of endosome to plasma membrane protein transport [GO:1905751] Relationships: is a type of positive regulation of intracellular transport [GO:0032388]; is a type of regulation of intracellular protein transport [GO:0033157]; is a type of positive regulation of protein transport [GO:0051222]; positively regulates intracellular protein transport [GO:0006886] Sources: GOC:tb Definition: Any process that activates or increases the frequency, rate or extent of the directed movement of proteins within cells.